{
  "gene_symbol": "ABCC5",
  "gene": "UniProtKB:O15440",
  "term_id": "GO:0055085",
  "term_label": "transmembrane transport",
  "gene_name": "ATP-binding cassette sub-family C member 5"
}